{
  "term_id": "UNKNOWN:0003",
  "gene": "UniProtKB:Q569K6",
  "term_label": "Unknown cellular component",
  "gene_symbol": "CCDC157",
  "gene_name": "Coiled-coil domain-containing protein 157"
}